{
  "term_label": "cytosol",
  "gene_name": "Ubiquilin-4",
  "gene_symbol": "UBQLN4",
  "gene": "UniProtKB:Q9NRR5",
  "term_id": "GO:0005829"
}